positive regulation of cellular response to insulin stimulus [GO:1900078] (biological process) Definition: Any process that activates or increases the frequency, rate or extent of cellular response to insulin stimulus. Relationships: is a type of positive regulation of cellular process [GO:0048522]; is a type of positive regulation of response to stimulus [GO:0048584]; is a type of GO:1900076; positively regulates cellular response to insulin stimulus [GO:0032869] Also known as: up regulation of cellular response to insulin stimulus, up-regulation of cellular response to insulin stimulus, upregulation of cellular response to insulin stimulus, activation of cellular response to insulin stimulus Sources: GOC:TermGenie, GOC:yaf Subtypes: positive regulation of insulin receptor signaling pathway [GO:0046628]